{
  "gene_name": "Annexin A3",
  "gene_symbol": "ANXA3",
  "term_id": "GO:0001786",
  "term_label": "phosphatidylserine binding",
  "gene": "UniProtKB:P12429"
}